{
  "gene_name": "RNA_RNP complex-1-interacting phosphatase",
  "gene": "UniProtKB:O75319",
  "term_label": "Unknown cellular component",
  "term_id": "UNKNOWN:0003",
  "gene_symbol": "DUSP11"
}